laminin-4 complex [GO:0005609] (cellular component) Definition: A laminin complex composed of alpha2, beta2 and gamma1 polypeptide chains. Relationships: is a type of laminin complex [GO:0043256] References: PMID:10842354 Sources: GOC:jl Also known as: laminin-221 complex